pyrrolysyl-tRNA synthetase activity [GO:0043767] (molecular function) Relationships: is_a aminoacyl-tRNA ligase activity [GO:0004812] References: PMID:15314242 Sources: RHEA:19277 Also known as: PylRS, pyrrolysine-tRNA ligase activity Definition: Catalysis of the reaction: ATP + L-pyrrolysine + tRNA(Pyl) = AMP + diphosphate + L-pyrrolysyl-tRNA(Pyl).